{
  "gene": "UniProtKB:A6NM43",
  "gene_symbol": "CCT8L1P",
  "term_label": "unfolded protein binding",
  "term_id": "GO:0051082",
  "gene_name": "Putative T-complex protein 1 subunit theta-like 1"
}